regulation of antibacterial peptide secretion [GO:0002797] (biological process) Sources: GOC:add Definition: Any process that modulates the frequency, rate, or extent of antibacterial peptide secretion. Relationships: is a type of regulation of antibacterial peptide production [GO:0002786]; is a type of GO:0002794; regulates antibacterial peptide secretion [GO:0002779] Subtypes: negative regulation of antibacterial peptide secretion [GO:0002798], positive regulation of antibacterial peptide secretion [GO:0002799]